{
  "gene_symbol": "NLGN3",
  "gene_name": "Neuroligin-3",
  "term_id": "GO:0005886",
  "gene": "UniProtKB:Q9NZ94",
  "term_label": "plasma membrane"
}